{
  "gene_symbol": "ZRANB1",
  "gene": "UniProtKB:Q9UGI0",
  "term_id": "GO:0070530",
  "term_label": "K63-linked polyubiquitin modification-dependent protein binding",
  "gene_name": "Ubiquitin thioesterase ZRANB1"
}